{
  "gene_symbol": "PHC1",
  "term_label": "negative regulation of DNA-templated transcription",
  "gene_name": "Polyhomeotic-like protein 1",
  "gene": "UniProtKB:P78364",
  "term_id": "GO:0045892"
}